{
  "gene_symbol": "KDR",
  "term_label": "endothelial cell differentiation",
  "term_id": "GO:0045446",
  "gene_name": "Vascular endothelial growth factor receptor 2",
  "gene": "UniProtKB:P35968"
}